{
  "term_id": "GO:0006898",
  "term_label": "receptor-mediated endocytosis",
  "gene_name": "Protein LMBR1L",
  "gene_symbol": "LMBR1L",
  "gene": "UniProtKB:Q6UX01"
}